{
  "term_id": "GO:0005886",
  "gene_name": "Cytoplasmic tyrosine-protein kinase BMX",
  "gene_symbol": "BMX",
  "term_label": "plasma membrane",
  "gene": "UniProtKB:P51813"
}